cell activation [GO:0001775] (BP) Definition: A multicellular organismal process by which exposure to an activating factor such as a cellular or soluble ligand results in a change in the morphology or behavior of a cell. Sources: GOC:mgi_curators Relationships: is a type of GO:0009987; is a type of multicellular organismal process [GO:0032501] Subtypes: cell activation involved in immune response [GO:0002263], follicular dendritic cell activation [GO:0002266], egg activation [GO:0007343], neuroblast activation [GO:0007407], GO:0014719, platelet activation [GO:0030168], keratinocyte activation [GO:0032980], GO:0042118, chondrocyte activation [GO:0044566], leukocyte activation [GO:0045321], glial cell activation [GO:0061900], GO:0071892, fibroblast activation [GO:0072537] Regulation: regulated by regulation of cell activation [GO:0050865]; negatively regulated by GO:0050866; positively regulated by GO:0050867